anther wall tapetum formation [GO:0048656] (biological process) Sources: GOC:jid, GOC:sm, GOC:tb Also known as: tapetal layer formation, tapetum formation Definition: The process that gives rise to the anther wall tapetum. This process pertains to the initial formation of a structure from unspecified parts. The anther wall tapetum is a layer of cells that provides a source of nutrition for the pollen grains as they mature. Relationships: is_a developmental process involved in reproduction [GO:0003006]; is a type of anatomical structure formation involved in morphogenesis [GO:0048646]; is part of stamen formation [GO:0048455]; is part of anther wall tapetum morphogenesis [GO:0048655]